NADP+ catabolic process [GO:0006742] (biological process) Relationships: is a type of GO:0006195; is a type of GO:0006739; is_a pyridine nucleotide catabolic process [GO:0019364] Definition: The chemical reactions and pathways resulting in the breakdown of nicotinamide adenine dinucleotide phosphate (NADP+), a coenzyme that interconverts with its reduced form, NADPH, in many redox and biosynthetic reactions. Also known as: NADP (oxidized) catabolic process, NADP (oxidized) catabolism, NADP (reduced) catabolic process, NADP (reduced) catabolism, NADP breakdown, NADP catabolic process, NADP catabolism, NADP degradation, NADPH catabolic process, NADPH catabolism, nicotinamide adenine dinucleotide phosphate catabolic process, nicotinamide adenine dinucleotide phosphate catabolism, oxidized NADP catabolic process, oxidized NADP catabolism, oxidized nicotinamide adenine dinucleotide phosphate catabolic process, oxidized nicotinamide adenine dinucleotide phosphate catabolism, reduced NADP catabolic process, reduced NADP catabolism, reduced nicotinamide adenine dinucleotide phosphate catabolic process, reduced nicotinamide adenine dinucleotide phosphate catabolism Sources: GOC:mah